N-succinylarginine dihydrolase activity [GO:0009015] (molecular function) Relationships: is a type of hydrolase activity, acting on carbon-nitrogen (but not peptide) bonds, in linear amidines [GO:0016813] Sources: EC:3.5.3.23, RHEA:19533 Also known as: N2-succinyl-L-arginine iminohydrolase (decarboxylating), N2-succinylarginine dihydrolase activity, arginine succinylhydrolase activity, succinylarginine dihydrolase activity, 2-N-succinyl-L-arginine iminohydrolase (decarboxylating), AruB, AstB, SADH Definition: Catalysis of the reaction: N(2)-succinyl-L-arginine + 2 H2O + 2 H+ = N(2)-succinyl-L-ornithine + CO2 + 2 NH4.